molybdopterin adenylyltransferase activity [GO:0061598] (molecular function) Sources: EC:2.7.7.75, GOC:dph Definition: Catalysis of the reaction ATP + molybdopterin = diphosphate + adenylyl-molybdopterin. Relationships: is a type of adenylyltransferase activity [GO:0070566]